inositol bisdiphosphate tetrakisphosphate diphosphatase activity [GO:0052841] (molecular function) Relationships: is a type of diphosphoinositol-polyphosphate diphosphatase activity [GO:0008486] Subtypes: inositol-1,5-bisdiphosphate-2,3,4,6-tetrakisphosphate 1-diphosphatase activity [GO:0052846], inositol-1,5-bisdiphosphate-2,3,4,6-tetrakisphosphate 5-diphosphatase activity [GO:0052847], inositol-3,5-bisdiphosphate-2,3,4,6-tetrakisphosphate 5-diphosphatase activity [GO:0052848] References: PMID:10827188, PMID:11502751 Definition: Catalysis of the reaction: bisdiphospho-1D-myo-inositol tetrakisphosphate + H2O = diphospho-1D-myo-inositol pentakisphosphate + phosphate.